{
  "term_label": "serine-type endopeptidase activity",
  "gene_symbol": "PRRG2",
  "gene": "UniProtKB:O14669",
  "term_id": "GO:0004252",
  "gene_name": "Transmembrane gamma-carboxyglutamic acid protein 2"
}